placenta blood vessel development [GO:0060674] (BP) Regulation: regulated by regulation of placenta blood vessel development [GO:0110079]; RO_0002213 by positive regulation of placenta blood vessel development [GO:0110080]; RO_0002212 by negative regulation of placenta blood vessel development [GO:0110081] Subtypes: labyrinthine layer blood vessel development [GO:0060716] References: PMID:16916377 Sources: GOC:dph Definition: The process whose specific outcome is the progression of a blood vessel of the placenta over time, from its formation to the mature structure. Relationships: is a type of blood vessel development [GO:0001568]; BFO_0000050 placenta development [GO:0001890]